negative regulation of meiotic spindle elongation [GO:1902120] (biological process) Definition: Any process that stops, prevents or reduces the frequency, rate or extent of meiotic spindle elongation. Relationships: is a type of negative regulation of meiotic nuclear division [GO:0045835]; is a type of regulation of meiotic spindle elongation [GO:1902119]; negatively regulates GO:0051232 References: PMID:23370392 Sources: GOC:TermGenie Also known as: down regulation of meiotic spindle elongation, down regulation of spindle elongation during meiosis, down-regulation of meiotic spindle elongation, down-regulation of spindle elongation during meiosis, downregulation of meiotic spindle elongation, downregulation of spindle elongation during meiosis, inhibition of spindle elongation during meiosis, negative regulation of spindle elongation during meiosis, inhibition of meiotic spindle elongation